{
  "gene_name": "Oxidized purine nucleoside triphosphate hydrolase",
  "term_label": "8-oxo-7,8-dihydroguanosine triphosphate pyrophosphatase activity",
  "gene_symbol": "NUDT1",
  "gene": "UniProtKB:P36639",
  "term_id": "GO:0008413"
}